{
  "gene_symbol": "ADA",
  "term_id": "GO:0046103",
  "gene_name": "Adenosine deaminase",
  "term_label": "inosine biosynthetic process",
  "gene": "UniProtKB:P00813"
}